{
  "term_label": "cytoplasm",
  "gene_name": "E3 ubiquitin-protein ligase RNF14",
  "gene": "UniProtKB:Q9UBS8",
  "gene_symbol": "RNF14",
  "term_id": "GO:0005737"
}